{
  "term_label": "cytoplasmic translation",
  "gene_name": "Large ribosomal subunit protein uL10",
  "gene": "UniProtKB:P05388",
  "gene_symbol": "RPLP0",
  "term_id": "GO:0002181"
}